{
  "gene": "UniProtKB:Q8N4N8",
  "gene_symbol": "KIF2B",
  "term_label": "cytoplasm",
  "gene_name": "Kinesin-like protein KIF2B",
  "term_id": "GO:0005737"
}